 [go#goslim:plant] Note: Plant GO slim